{
  "gene_symbol": "GABRA3",
  "gene": "UniProtKB:P34903",
  "gene_name": "Gamma-aminobutyric acid receptor subunit alpha-3",
  "term_label": "chloride channel activity",
  "term_id": "GO:0005254"
}